{
  "gene_name": "Exosome complex component RRP45",
  "gene": "UniProtKB:Q06265",
  "term_label": "nuclear mRNA surveillance",
  "gene_symbol": "EXOSC9",
  "term_id": "GO:0071028"
}